{
  "gene_name": "Zinc finger and BTB domain-containing protein 41",
  "gene_symbol": "ZBTB41",
  "gene": "UniProtKB:Q5SVQ8",
  "term_id": "UNKNOWN:0003",
  "term_label": "Unknown cellular component"
}